ERBB2-ERBB4 signaling pathway [GO:0038135] (biological process) References: PMID:16460914 Sources: GOC:signaling Also known as: ERBB2-ERBB4 signalling pathway, HER2-HER4 signaling pathway Definition: The series of molecular signals initiated by binding of a ligand to a ERBB4 receptor on the surface of a cell, followed by transmission of the signal by a heterodimeric complex of ERBB2 and ERBB4. ERBB2, which does not bind any known ligand, is activated through formation of a heterodimer with another ligand-activated ERBB family member such as ERBB4. Relationships: is a type of ERBB2 signaling pathway [GO:0038128]; is a type of ERBB4 signaling pathway [GO:0038130]